{
  "gene": "UniProtKB:Q9Y4Y9",
  "gene_symbol": "LSM5",
  "term_id": "GO:0000398",
  "gene_name": "U6 snRNA-associated Sm-like protein LSm5",
  "term_label": "mRNA splicing, via spliceosome"
}